{
  "gene_name": "C-X-C motif chemokine 5",
  "gene_symbol": "CXCL5",
  "gene": "UniProtKB:P42830",
  "term_id": "GO:0008009",
  "term_label": "chemokine activity"
}